{
  "gene": "UniProtKB:Q8IXF9",
  "term_id": "UNKNOWN:0002",
  "gene_name": "Aquaporin-12A",
  "gene_symbol": "AQP12A",
  "term_label": "Unknown biological process"
}